positive regulation of phospholipid efflux [GO:1902995] (biological process) Relationships: is a type of GO:1902994; is a type of GO:2001140; positively regulates phospholipid efflux [GO:0033700] Also known as: positive regulation of phospholipid export, up regulation of phospholipid efflux, up regulation of phospholipid export, up-regulation of phospholipid efflux, up-regulation of phospholipid export, upregulation of phospholipid efflux, upregulation of phospholipid export, activation of phospholipid efflux, activation of phospholipid export References: PMID:12042316 Sources: GOC:TermGenie, GOC:sjp, GO_REF:0000058 Definition: Any process that activates or increases the frequency, rate or extent of phospholipid efflux.